{
  "gene_name": "Polyadenylate-binding protein 4",
  "gene_symbol": "PABPC4",
  "term_id": "GO:0008266",
  "gene": "UniProtKB:Q13310",
  "term_label": "poly(U) RNA binding"
}